{
  "gene": "UniProtKB:Q9BUK0",
  "term_label": "mitochondrial respiratory chain complex assembly",
  "term_id": "GO:0033108",
  "gene_symbol": "CHCHD7",
  "gene_name": "Coiled-coil-helix-coiled-coil-helix domain-containing protein 7"
}